{
  "gene": "UniProtKB:Q9UN37",
  "gene_symbol": "VPS4A",
  "term_label": "ubiquitin-independent protein catabolic process via the multivesicular body sorting pathway",
  "gene_name": "Vacuolar protein sorting-associated protein 4A",
  "term_id": "GO:0090611"
}